{
  "gene_name": "Proliferation-associated protein 2G4",
  "gene": "UniProtKB:Q9UQ80",
  "term_label": "Unknown biological process",
  "term_id": "UNKNOWN:0002",
  "gene_symbol": "PA2G4"
}